{
  "term_id": "GO:0061564",
  "gene_symbol": "NEFH",
  "gene_name": "Neurofilament heavy polypeptide",
  "gene": "UniProtKB:P12036",
  "term_label": "axon development"
}